{
  "gene": "UniProtKB:P51861",
  "gene_symbol": "CDR1",
  "term_id": "UNKNOWN:0002",
  "gene_name": "Cerebellar degeneration-related antigen 1",
  "term_label": "Unknown biological process"
}